manganese import into cell [GO:0140967] (biological process) Also known as: manganese influx Relationships: is a type of manganese ion transmembrane transport [GO:0071421]; is a type of inorganic cation import across plasma membrane [GO:0098659] References: PMID:22773749 Definition: The directed movement of mangnanese ions from outside of a cell into a cell.